{
  "gene": "UniProtKB:Q9UPV9",
  "term_label": "neurogenesis",
  "term_id": "GO:0022008",
  "gene_symbol": "TRAK1",
  "gene_name": "Trafficking kinesin-binding protein 1"
}